{
  "term_id": "GO:0003713",
  "gene": "UniProtKB:Q16594",
  "gene_name": "Transcription initiation factor TFIID subunit 9",
  "gene_symbol": "TAF9",
  "term_label": "transcription coactivator activity"
}